{
  "gene_name": "Vasopressin V1b receptor",
  "term_label": "cellular response to hormone stimulus",
  "gene_symbol": "AVPR1B",
  "gene": "UniProtKB:P47901",
  "term_id": "GO:0032870"
}